{
  "gene_symbol": "PAX4",
  "gene_name": "Paired box protein Pax-4",
  "term_label": "brain development",
  "term_id": "GO:0007420",
  "gene": "UniProtKB:O43316"
}